{
  "gene": "UniProtKB:O76064",
  "term_id": "GO:0000151",
  "gene_symbol": "RNF8",
  "term_label": "ubiquitin ligase complex",
  "gene_name": "E3 ubiquitin-protein ligase RNF8"
}